SMN-Sm protein complex [GO:0034719] (cellular component) Subtypes: GO:0034730, Lsm-containing SMN-Sm protein complex [GO:0034731] Relationships: is a type of GO:0120114; is part of cytoplasm [GO:0005737]; has part SMN complex [GO:0032797] References: PMID:11522829, PMID:17401408 Sources: GOC:vw Definition: A protein complex formed by the association of several methylated Sm proteins with the SMN complex; the latter contains the survival motor neuron (SMN) protein and at least eight additional integral components, including the Gemin2-8 and unrip proteins; additional proteins, including galectin-1 and galectin-3, are also found in the SMN-SM complex. The SMN-Sm complex is involved in spliceosomal snRNP assembly in the cytoplasm. Note: Note that this complex is sometimes referred to as the 'SMN complex', but it should not be confused with GO:0032797. Also known as: SMN-containing protein complex